{
  "term_id": "GO:0005615",
  "term_label": "extracellular space",
  "gene_name": "Augurin",
  "gene_symbol": "ECRG4",
  "gene": "UniProtKB:Q9H1Z8"
}